MHC class II protein complex assembly [GO:0002399] (biological process) Relationships: is a type of MHC protein complex assembly [GO:0002396] Definition: The aggregation, arrangement and bonding together of a set of components to form an MHC class II protein complex. References: PMID:15771591 Sources: GOC:add, ISBN:0781735149